{
  "gene": "UniProtKB:Q8TEC5",
  "term_label": "ubiquitin protein ligase activity",
  "gene_symbol": "SH3RF2",
  "gene_name": "E3 ubiquitin-protein ligase SH3RF2",
  "term_id": "GO:0061630"
}